{
  "gene_symbol": "GUSBP11",
  "gene": "UniProtKB:Q6P575",
  "term_id": "UNKNOWN:0003",
  "gene_name": "Putative inactive beta-glucuronidase protein GUSBP11",
  "term_label": "Unknown cellular component"
}